{
  "gene_name": "Keratin, type I cytoskeletal 19",
  "term_id": "GO:0030280",
  "gene_symbol": "KRT19",
  "gene": "UniProtKB:P08727",
  "term_label": "structural constituent of skin epidermis"
}